{
  "gene": "UniProtKB:Q9HC16",
  "gene_name": "DNA dC-dU-editing enzyme APOBEC-3G",
  "term_id": "GO:0045869",
  "gene_symbol": "APOBEC3G",
  "term_label": "negative regulation of single stranded viral RNA replication via double stranded DNA intermediate"
}